{
  "gene": "UniProtKB:Q9NXS3",
  "gene_symbol": "KLHL28",
  "term_id": "GO:0031463",
  "gene_name": "Kelch-like protein 28",
  "term_label": "Cul3-RING ubiquitin ligase complex"
}